{
  "gene_symbol": "UBE2J1",
  "gene": "UniProtKB:Q9Y385",
  "gene_name": "Ubiquitin-conjugating enzyme E2 J1",
  "term_label": "ERAD pathway",
  "term_id": "GO:0036503"
}